{
  "gene": "UniProtKB:P33981",
  "term_id": "GO:0004674",
  "gene_symbol": "TTK",
  "term_label": "protein serine/threonine kinase activity",
  "gene_name": "Dual specificity protein kinase TTK"
}